{
  "term_label": "sequence-specific DNA binding",
  "gene_name": "E3 SUMO-protein ligase ZNF451",
  "term_id": "GO:0043565",
  "gene": "UniProtKB:Q9Y4E5",
  "gene_symbol": "ZNF451"
}